{
  "gene": "UniProtKB:Q9HAI6",
  "term_id": "UNKNOWN:0003",
  "term_label": "Unknown cellular component",
  "gene_name": "TLR adapter interacting with SLC15A4 on the lysosome",
  "gene_symbol": "TASL"
}